glutathione disulfide oxidoreductase activity [GO:0015038] (molecular function) Definition: Catalysis of the reaction: 2 glutathione + electron acceptor = glutathione disulfide + electron donor. Also known as: glutaredoxin, glutathione oxidoreductase activity, glutathione disulphide oxidoreductase activity Sources: GOC:mah Subtypes: glutathione-disulfide reductase (NADPH) activity [GO:0004362], GO:0045174 Relationships: is a type of GO:0015036